{
  "term_label": "L-phenylalanine catabolic process",
  "gene": "UniProtKB:P00439",
  "gene_name": "Phenylalanine-4-hydroxylase",
  "gene_symbol": "PAH",
  "term_id": "GO:0006559"
}